{
  "gene": "UniProtKB:Q6ZMJ2",
  "gene_symbol": "SCARA5",
  "term_id": "GO:0005886",
  "gene_name": "Scavenger receptor class A member 5",
  "term_label": "plasma membrane"
}